{
  "gene_name": "F-box only protein 2",
  "term_label": "SCF ubiquitin ligase complex",
  "term_id": "GO:0019005",
  "gene_symbol": "FBXO2",
  "gene": "UniProtKB:Q9UK22"
}